{
  "term_id": "UNKNOWN:0001",
  "term_label": "Unknown molecular function",
  "gene": "UniProtKB:B6SEH8",
  "gene_name": "Endogenous retrovirus group V member 1 Env polyprotein",
  "gene_symbol": "ERVV-1"
}